polyketide catabolic process [GO:0030640] (biological process) Definition: The chemical reactions and pathways resulting in the breakdown of polyketides, any of a diverse group of natural products synthesized via linear poly-beta-ketones, which are themselves formed by repetitive head-to-tail addition of acetyl (or substituted acetyl) units indirectly derived from acetate (or a substituted acetate) by a mechanism similar to that for fatty acid biosynthesis but without the intermediate reductive steps. Subtypes: enterobactin catabolic process [GO:0046214], asperfuranone catabolic process [GO:1900553], GO:1900610, F-9775B catabolic process [GO:1900613], averantin catabolic process [GO:1900762], fonsecin catabolic process [GO:1900768], tetracenomycin C catabolic process [GO:1901105], granaticin catabolic process [GO:1901108], erythromycin catabolic process [GO:1901114], GO:1901517, aspyridone B catabolic process [GO:1901520], oxytetracycline catabolic process [GO:1901762], daunorubicin catabolic process [GO:1901770], neosartoricin catabolic process [GO:1902049] Sources: GOC:mah, ISBN:0198506732 Relationships: is a type of polyketide metabolic process [GO:0030638]; is a type of secondary metabolite catabolic process [GO:0090487] Also known as: polyketide breakdown, polyketide catabolism, polyketide degradation